{
  "gene_name": "Folylpolyglutamate synthase, mitochondrial",
  "gene_symbol": "FPGS",
  "term_id": "GO:0046901",
  "gene": "UniProtKB:Q05932",
  "term_label": "tetrahydrofolylpolyglutamate biosynthetic process"
}